{
  "term_label": "C-C chemokine receptor activity",
  "gene_symbol": "CXCR5",
  "gene": "UniProtKB:P32302",
  "term_id": "GO:0016493",
  "gene_name": "C-X-C chemokine receptor type 5"
}